sprouting of injured axon [GO:0048682] (biological process) Subtypes: collateral sprouting of injured axon [GO:0048674], axon extension involved in regeneration [GO:0048677], formation of growth cone in injured axon [GO:0048689] Relationships: is a type of developmental cell growth [GO:0048588]; is a type of GO:0060560; BFO_0000050 axon regeneration [GO:0031103] Definition: The process involved in sprouting of an injured axon. Sources: GOC:dgh, GOC:dph, GOC:jid, GOC:lm Regulation: regulated by GO:0048686; positively regulated by positive regulation of sprouting of injured axon [GO:0048687]; negatively regulated by GO:0048688